cytoophidium [GO:0097268] (cellular component) Definition: A filamentous, membrane-less subcellular structure composed primarily of polymerized metabolic enzymes, most notably cytidine triphosphate synthase (CTPS). Cytoophidia are evolutionarily conserved structures found across archaea, bacteria, and eukaryotes. References: PMID:20513629, PMID:21930098, PMID:37248970 Sources: Wikipedia:CTP_synthase#Cytoophidium Relationships: is a type of GO:0099512